(R)-3-amino-2-methylpropionate-pyruvate transaminase activity [GO:0047305] (molecular function) Definition: Catalysis of the reaction: (2R)-3-amino-2-methylpropanoate + pyruvate = 2-methyl-3-oxopropanoate + L-alanine. Sources: EC:2.6.1.40, RHEA:18393 Also known as: (R)-3-amino-2-methylpropanoate aminotransferase activity, (R)-3-amino-2-methylpropanoate transaminase activity, (R)-3-amino-2-methylpropionate transaminase activity, (R)-3-amino-2-methylpropionate-pyruvate aminotransferase activity, (R)-3-amino-2-methylpropanoate:pyruvate aminotransferase activity, (R)-3-amino-2-methylpropionate--pyruvate aminotransferase activity, D-3-aminoisobutyrate--pyruvate aminotransferase activity, D-3-aminoisobutyrate--pyruvate transaminase activity, D-3-aminoisobutyrate-pyruvate transaminase activity, D-AIBAT activity, D-beta-aminoisobutyrate:pyruvate aminotransferase activity, beta-aminoisobutyrate--pyruvate transaminase activity, beta-aminoisobutyrate-pyruvate aminotransferase activity Note: Note that this function was EC:2.6.1.61. Relationships: is_a transaminase activity [GO:0008483]